negative regulation of female receptivity [GO:0007621] (biological process) Definition: Any process that stops, prevents or reduces the receptiveness of a female to male advances. References: PMID:11092827 Sources: GOC:bf Also known as: down regulation of female receptivity, down-regulation of female receptivity, downregulation of female receptivity, inhibition of female receptivity Relationships: is a type of regulation of female receptivity [GO:0045924] Subtypes: negative regulation of female receptivity, post-mating [GO:0045434]